epithelial cell migration, open tracheal system [GO:0007427] (biological process) Also known as: tracheal cell migration, tracheal epithelial cell migration Sources: GOC:bf, GOC:mtg_sensu Regulation: regulated by regulation of epithelial cell migration, open tracheal system [GO:2000274] Definition: The orderly movement of epithelial cells during development of an open tracheal system. An example of this is found in Drosophila melanogaster. Relationships: is a type of GO:0010631; is part of open tracheal system development [GO:0007424]